extrinsic component of synaptic membrane [GO:0099243] (cellular component) Relationships: is a type of GO:0019897; is part of GO:0097060 Sources: GOC:dos Subtypes: extrinsic component of presynaptic membrane [GO:0098888], extrinsic component of postsynaptic membrane [GO:0098890] Definition: The component of the synaptic membrane consisting of gene products and protein complexes that are loosely bound to one of its surfaces, but not integrated into the hydrophobic region.